negative regulation of ATP metabolic process [GO:1903579] (biological process) Relationships: is a type of negative regulation of purine nucleotide metabolic process [GO:1900543]; is a type of regulation of ATP metabolic process [GO:1903578]; negatively regulates ATP metabolic process [GO:0046034] Definition: Any process that stops, prevents or reduces the frequency, rate or extent of ATP metabolic process. Also known as: down regulation of ATP metabolic process, down regulation of ATP metabolism, down-regulation of ATP metabolic process, down-regulation of ATP metabolism, downregulation of ATP metabolic process, downregulation of ATP metabolism, negative regulation of ATP metabolism, inhibition of ATP metabolic process, inhibition of ATP metabolism References: PMID:20695849 Sources: GOC:TermGenie, GO_REF:0000058 Subtypes: negative regulation of glycolytic process [GO:0045820], negative regulation of ATP biosynthetic process [GO:2001170]